{
  "term_label": "microtubule",
  "gene_symbol": "MX1",
  "gene_name": "Interferon-induced GTP-binding protein Mx1",
  "term_id": "GO:0005874",
  "gene": "UniProtKB:P20591"
}